{
  "gene": "UniProtKB:P0C7M7",
  "gene_symbol": "ACSM4",
  "gene_name": "Acyl-coenzyme A synthetase ACSM4, mitochondrial",
  "term_label": "fatty-acyl-CoA synthase activity",
  "term_id": "GO:0004321"
}